{
  "term_label": "Unknown cellular component",
  "gene": "UniProtKB:Q9BQ49",
  "term_id": "UNKNOWN:0003",
  "gene_symbol": "SMIM7",
  "gene_name": "Small integral membrane protein 7"
}